ribonuclease A activity [GO:0004522] (molecular function) Definition: Catalysis of the endonucleolytic cleavage of RNA to 3'-phosphomononucleotides and 3'-phosphooligonucleotides ending in C-P or U-P with 2',3'-cyclic phosphate intermediates. Also known as: RNase activity, alkaline ribonuclease activity, ceratitis capitata alkaline ribonuclease activity, ribonucleate 3'-pyrimidino-oligonucleotidohydrolase activity, ribonucleic phosphatase activity, pancreatic ribonuclease activity, RNase A activity, RNase I activity, S-genotype-assocd. glycoproteins, SLSG glycoproteins, endoribonuclease I, gene S glycoproteins, gene S locus-specific glycoproteins, pancreatic RNase activity, ribonuclease I activity Sources: EC:4.6.1.18 Relationships: is a type of RNA endonuclease activity [GO:0004521]; is a type of GO:0016849